root cap development [GO:0048829] (biological process) Definition: The process whose specific outcome is the progression of the root cap over time, from its formation to the mature structure. The root cap protects the root meristem from friction as the root grows through the soil. The cap is made up of a group of parenchyma cells which secrete a glycoprotein mucilage as a lubricant. Relationships: is a type of anatomical structure development [GO:0048856]; is part of root development [GO:0048364] Sources: GOC:tb